{
  "term_id": "GO:0007340",
  "gene_symbol": "TRIM36",
  "term_label": "acrosome reaction",
  "gene": "UniProtKB:Q9NQ86",
  "gene_name": "E3 ubiquitin-protein ligase TRIM36"
}